{
  "term_id": "GO:0031683",
  "term_label": "G-protein beta/gamma-subunit complex binding",
  "gene_name": "Guanine nucleotide-binding protein G(t) subunit alpha-2",
  "gene_symbol": "GNAT2",
  "gene": "UniProtKB:P19087"
}